trachea morphogenesis [GO:0060439] (biological process) Relationships: is a type of animal organ morphogenesis [GO:0009887]; is part of trachea development [GO:0060438] Sources: GOC:dph Definition: The process in which a trachea is generated and organized. The trachea is the portion of the airway that attaches to the bronchi as it branches.